{
  "gene_name": "Cilia- and flagella-associated protein 57",
  "gene": "UniProtKB:Q96MR6",
  "gene_symbol": "CFAP57",
  "term_label": "Unknown cellular component",
  "term_id": "UNKNOWN:0003"
}